tartrate transmembrane transporter activity [GO:0015554] (molecular function) Subtypes: tartrate:succinate antiporter activity [GO:0015516] Definition: Enables the transfer of tartrate from one side of a membrane to the other. Tartrate is the anion of 2,3-dihydroxybutanedioic acid, one of the aldaric acids. The L(+) enantiomer occurs widely in plants, especially in grape juice, and in fungi and bacteria. Relationships: is_a salt transmembrane transporter activity [GO:1901702] Sources: GOC:ai